{
  "gene_name": "Cardiac phospholamban",
  "term_id": "GO:1902081",
  "term_label": "negative regulation of calcium ion import into sarcoplasmic reticulum",
  "gene": "UniProtKB:P26678",
  "gene_symbol": "PLN"
}